positive regulation of calcium-dependent ATPase activity [GO:1903612] (biological process) Relationships: is a type of positive regulation of ATP-dependent activity [GO:0032781]; positively regulates calcium-dependent ATPase activity [GO:0030899] Also known as: up regulation of calcium-dependent ATPase activity, up-regulation of calcium-dependent ATPase activity, upregulation of calcium-dependent ATPase activity, activation of calcium-dependent ATPase activity Definition: Any process that activates or increases the frequency, rate or extent of calcium-dependent ATPase activity. References: PMID:10861851 Sources: GOC:TermGenie, GO_REF:0000059